{
  "gene_symbol": "RANGAP1",
  "term_id": "GO:0051168",
  "term_label": "nuclear export",
  "gene": "UniProtKB:P46060",
  "gene_name": "Ran GTPase-activating protein 1"
}